{
  "gene_name": "CMP-N-acetylneuraminate-beta-galactosamide-alpha-2,3-sialyltransferase 2",
  "gene": "UniProtKB:Q16842",
  "term_label": "membrane",
  "term_id": "GO:0016020",
  "gene_symbol": "ST3GAL2"
}